{
  "gene": "UniProtKB:Q8TBZ6",
  "gene_name": "tRNA methyltransferase 10 homolog A",
  "gene_symbol": "TRMT10A",
  "term_id": "GO:0002939",
  "term_label": "tRNA N1-guanine methylation"
}